{
  "gene_symbol": "IL2RG",
  "gene": "UniProtKB:P31785",
  "gene_name": "Cytokine receptor common subunit gamma",
  "term_id": "GO:0043235",
  "term_label": "receptor complex"
}